{
  "term_label": "T cell activation involved in immune response",
  "gene_symbol": "IFNA1",
  "gene_name": "Interferon alpha-1_13",
  "term_id": "GO:0002286",
  "gene": "UniProtKB:P01562"
}